{
  "gene": "UniProtKB:O94979",
  "gene_symbol": "SEC31A",
  "term_id": "GO:0070971",
  "term_label": "endoplasmic reticulum exit site",
  "gene_name": "Protein transport protein Sec31A"
}